TAP1 binding [GO:0046978] (molecular function) References: PMID:11133832 Relationships: is a type of TAP binding [GO:0046977] Definition: Binding to the TAP1 subunit of TAP (transporter associated with antigen processing) protein.